{
  "gene_name": "Homeobox domain-containing protein",
  "term_id": "GO:0000977",
  "term_label": "RNA polymerase II transcription regulatory region sequence-specific DNA binding",
  "gene_symbol": "LOC124905412",
  "gene": "UniProtKB:A0A1B0GW55"
}